{
  "term_id": "GO:0032433",
  "gene_symbol": "MYO3B",
  "term_label": "filopodium tip",
  "gene": "UniProtKB:Q8WXR4",
  "gene_name": "Myosin-IIIb"
}